{
  "term_id": "GO:2001238",
  "gene_symbol": "LTB",
  "gene": "UniProtKB:Q06643",
  "term_label": "positive regulation of extrinsic apoptotic signaling pathway",
  "gene_name": "Lymphotoxin-beta"
}